positive regulation of long-term neuronal synaptic plasticity [GO:0048170] (biological process) Also known as: up regulation of long-term neuronal synaptic plasticity, up-regulation of long-term neuronal synaptic plasticity, upregulation of long-term neuronal synaptic plasticity, activation of long-term neuronal synaptic plasticity, stimulation of long-term neuronal synaptic plasticity Note: Note that the syntax of the definition of this term is different from the usual regulation syntax because it describes regulation of a trait rather than regulation of a process. Definition: A process that increases long-term neuronal synaptic plasticity, the ability of neuronal synapses to change long-term as circumstances require. Long-term neuronal synaptic plasticity generally involves increase or decrease in actual synapse numbers. References: PMID:11891290 Sources: GOC:jid Relationships: is a type of regulation of long-term neuronal synaptic plasticity [GO:0048169]; is a type of positive regulation of neurogenesis [GO:0050769]